{
  "term_id": "UNKNOWN:0002",
  "gene": "UniProtKB:Q9H0P0",
  "term_label": "Unknown biological process",
  "gene_symbol": "NT5C3A",
  "gene_name": "Cytosolic 5'-nucleotidase 3A"
}